cellular response to lipoteichoic acid [GO:0071223] (biological process) Definition: Any process that results in a change in state or activity of a cell (in terms of movement, secretion, enzyme production, gene expression, etc.) as a result of a lipoteichoic acid stimulus; lipoteichoic acid is a major component of the cell wall of gram-positive bacteria and typically consists of a chain of glycerol-phosphate repeating units linked to a glycolipid anchor. Also known as: cellular response to LTA Sources: GOC:mah Relationships: is a type of response to lipoteichoic acid [GO:0070391]; is a type of GO:0071219; is a type of cellular response to oxygen-containing compound [GO:1901701]